{
  "gene_symbol": "PGF",
  "term_label": "growth factor activity",
  "term_id": "GO:0008083",
  "gene_name": "Placenta growth factor",
  "gene": "UniProtKB:P49763"
}